{
  "gene": "UniProtKB:Q15853",
  "gene_symbol": "USF2",
  "term_label": "Unknown cellular component",
  "term_id": "UNKNOWN:0003",
  "gene_name": "Upstream stimulatory factor 2"
}